{
  "gene_name": "Tight junction protein ZO-2",
  "gene_symbol": "TJP2",
  "term_id": "GO:0005886",
  "gene": "UniProtKB:Q9UDY2",
  "term_label": "plasma membrane"
}